{
  "term_id": "GO:0004930",
  "term_label": "G protein-coupled receptor activity",
  "gene": "UniProtKB:Q9BX74",
  "gene_name": "TM2 domain-containing protein 1",
  "gene_symbol": "TM2D1"
}